{
  "gene_name": "Taste receptor type 2 member 60",
  "term_label": "Unknown molecular function",
  "gene": "UniProtKB:P59551",
  "term_id": "UNKNOWN:0001",
  "gene_symbol": "TAS2R60"
}